cell migration involved in gastrulation [GO:0042074] (BP) Subtypes: mesoderm migration involved in gastrulation [GO:0007509], ingression involved in gastrulation with mouth forming second [GO:0055111], GO:0060030, mediolateral intercalation [GO:0060031], cell migration involved in mesendoderm migration [GO:0090134] References: PMID:16099638 Sources: GOC:jl Definition: The migration of individual cells within the blastocyst to help establish the multi-layered body plan of the organism (gastrulation). For example, the migration of cells from the surface to the interior of the embryo (ingression). Relationships: is a type of ameboidal-type cell migration [GO:0001667]; is part of gastrulation [GO:0007369]